{
  "term_id": "UNKNOWN:0002",
  "gene_name": "Apolipoprotein L5",
  "term_label": "Unknown biological process",
  "gene_symbol": "APOL5",
  "gene": "UniProtKB:Q9BWW9"
}